{
  "term_label": "cytoplasm",
  "gene": "UniProtKB:P14618",
  "term_id": "GO:0005737",
  "gene_name": "Pyruvate kinase PKM",
  "gene_symbol": "PKM"
}